{
  "gene_symbol": "LRRC8B",
  "term_label": "Unknown molecular function",
  "term_id": "UNKNOWN:0001",
  "gene": "UniProtKB:Q6P9F7",
  "gene_name": "Volume-regulated anion channel subunit LRRC8B"
}